{
  "gene": "UniProtKB:Q9UJX3",
  "term_label": "enzyme-substrate adaptor activity",
  "gene_name": "Anaphase-promoting complex subunit 7",
  "gene_symbol": "ANAPC7",
  "term_id": "GO:0140767"
}